{
  "gene_name": "SPARC-related modular calcium-binding protein 1",
  "gene": "UniProtKB:Q9H4F8",
  "term_id": "GO:0005604",
  "gene_symbol": "SMOC1",
  "term_label": "basement membrane"
}